{
  "gene_symbol": "GATA5",
  "term_id": "GO:0000981",
  "gene": "UniProtKB:Q9BWX5",
  "gene_name": "Transcription factor GATA-5",
  "term_label": "DNA-binding transcription factor activity, RNA polymerase II-specific"
}